3-hydroxyisobutyrate dehydrogenase activity [GO:0008442] (molecular function) Definition: Catalysis of the reaction: 3-hydroxy-2-methylpropanoate + NAD+ = 2-methyl-3-oxopropanoate + NADH + H+. Relationships: is a type of oxidoreductase activity, acting on the CH-OH group of donors, NAD or NADP as acceptor [GO:0016616] Sources: EC:1.1.1.31